{
  "gene": "UniProtKB:Q96C92",
  "term_id": "GO:0005813",
  "term_label": "centrosome",
  "gene_name": "Endosome-associated-trafficking regulator 1",
  "gene_symbol": "ENTR1"
}